{
  "gene_symbol": "OR4A4P",
  "gene_name": "Putative olfactory receptor 4A4",
  "term_id": "GO:0004984",
  "gene": "UniProtKB:Q8NGN8",
  "term_label": "olfactory receptor activity"
}